{
  "gene_name": "DNA polymerase theta",
  "gene_symbol": "POLQ",
  "gene": "UniProtKB:O75417",
  "term_label": "double-strand break repair via alternative nonhomologous end joining",
  "term_id": "GO:0097681"
}